{
  "term_id": "GO:0006527",
  "gene_symbol": "NOS3",
  "gene_name": "Nitric oxide synthase 3",
  "term_label": "L-arginine catabolic process",
  "gene": "UniProtKB:P29474"
}